{
  "gene_symbol": "KIR2DS2",
  "gene": "UniProtKB:P43631",
  "gene_name": "Killer cell immunoglobulin-like receptor 2DS2",
  "term_label": "transmembrane signaling receptor activity",
  "term_id": "GO:0004888"
}